{
  "gene": "UniProtKB:Q6ZQR2",
  "term_id": "UNKNOWN:0001",
  "gene_name": "Cilia- and flagella-associated protein 77",
  "gene_symbol": "CFAP77",
  "term_label": "Unknown molecular function"
}